initiation of dorsal closure [GO:0007392] (biological process) Definition: Events that occur at the start of dorsal closure. Sources: GOC:bf Relationships: is_a embryonic morphogenesis [GO:0048598]; is part of dorsal closure [GO:0007391]